{
  "gene_symbol": "COX6C",
  "term_id": "UNKNOWN:0001",
  "gene": "UniProtKB:P09669",
  "gene_name": "Cytochrome c oxidase subunit 6C",
  "term_label": "Unknown molecular function"
}